trans-synaptic signaling by BDNF, modulating synaptic transmission [GO:0099183] (biological process) Note: Note that this term was created for the SynGO project, and will be obsoleted when the SynGO annotations are made in Noctua. Regulation: regulated by regulation of trans-synaptic signaling by BDNF, modulating synaptic transmission [GO:0150035] Relationships: is a type of GO:0099191; is a type of GO:0099550 Definition: Cell-cell signaling between presynapse and postsynapse, via the vesicular release and reception of brain derived neurotrophic factor (BDNF), that modulates the synaptic transmission properties of the synapse. Sources: GOC:dos